{
  "gene_name": "Probable dolichyl pyrophosphate Glc1Man9GlcNAc2 alpha-1,3-glucosyltransferase",
  "gene_symbol": "ALG8",
  "term_label": "endoplasmic reticulum membrane",
  "gene": "UniProtKB:Q9BVK2",
  "term_id": "GO:0005789"
}